negative regulation of parathyroid hormone secretion [GO:2000829] (BP) Definition: Any process that stops, prevents or reduces the frequency, rate or extent of parathyroid hormone secretion. Also known as: negative regulation of PTH secretion, negative regulation of parathormone secretion, negative regulation of parathyrin secretion Sources: GOC:obol Relationships: is a type of negative regulation of hormone secretion [GO:0046888]; is a type of negative regulation of multicellular organismal process [GO:0051241]; is a type of regulation of parathyroid hormone secretion [GO:2000828]; negatively regulates parathyroid hormone secretion [GO:0035898]